multi-multicellular organism process [GO:0044706] (biological process) Sources: GOC:jl Definition: A multicellular organism process which involves another multicellular organism of the same or different species. Subtypes: insemination [GO:0007320], GO:0007341, female pregnancy [GO:0007565], GO:0007567, sperm competition [GO:0046692], GO:0048624, GO:0060378 Relationships: is a type of GO:0032501